inositol-1,3,4-trisphosphate 6-kinase activity [GO:0052725] (molecular function) Also known as: 1D-myo-inositol-trisphosphate 6-kinase activity, IP3 6-kinase activity, inositol-trisphosphate 6-kinase activity, inositol 1,3,4-trisphosphate 6-kinase activity, Ins(1,3,4)P3 6-kinase activity, ins(1,3,4)P(3) 6-kinase activity Sources: RHEA:20940 Relationships: is a type of inositol trisphosphate kinase activity [GO:0051766] Definition: Catalysis of the reaction: 1D-myo-inositol 1,3,4-trisphosphate + ATP = 1D-myo-inositol 1,3,4,6-tetrakisphosphate + ADP + H+.